{
  "gene_name": "A disintegrin and metalloproteinase with thrombospondin motifs 2",
  "gene": "UniProtKB:O95450",
  "term_label": "proteolysis",
  "gene_symbol": "ADAMTS2",
  "term_id": "GO:0006508"
}